{
  "gene": "UniProtKB:H3BV12",
  "term_id": "GO:0007030",
  "gene_symbol": "GOLGA8Q",
  "gene_name": "Golgin subfamily A member 8Q",
  "term_label": "Golgi organization"
}